{
  "term_id": "UNKNOWN:0003",
  "term_label": "Unknown cellular component",
  "gene_symbol": "RIMS4",
  "gene": "UniProtKB:Q9H426",
  "gene_name": "Regulating synaptic membrane exocytosis protein 4"
}